{
  "gene_symbol": "TNFRSF21",
  "gene_name": "Tumor necrosis factor receptor superfamily member 21",
  "gene": "UniProtKB:O75509",
  "term_label": "adaptive immune response",
  "term_id": "GO:0002250"
}